alphaV-beta3 integrin-LPP3 complex [GO:0071129] (cellular component) Definition: A protein complex that consists of an alphaV-beta3 integrin complex bound to lipid phosphate phosphohydrolase-3. References: PMID:16099422 Also known as: ITGAV-ITGB3-PPAP2B complex Relationships: is a type of GO:0098797